trachea cartilage morphogenesis [GO:0060535] (biological process) Definition: The process in which the anatomical structures of cartilage in the trachea are generated and organized. Relationships: is_a cartilage morphogenesis [GO:0060536]; is part of GO:0060439; is part of trachea cartilage development [GO:0060534] Sources: GOC:dph